{
  "term_label": "G protein-coupled receptor signaling pathway",
  "term_id": "GO:0007186",
  "gene": "UniProtKB:Q8NG41",
  "gene_symbol": "NPB",
  "gene_name": "Neuropeptide B"
}